{
  "gene": "UniProtKB:Q13508",
  "gene_name": "Ecto-ADP-ribosyltransferase 3",
  "gene_symbol": "ART3",
  "term_id": "UNKNOWN:0003",
  "term_label": "Unknown cellular component"
}